{
  "term_label": "early endosome",
  "gene_symbol": "WASH4P",
  "gene": "UniProtKB:A8MWX3",
  "gene_name": "Putative WAS protein family homolog 4",
  "term_id": "GO:0005769"
}